{
  "gene_name": "Autophagy-related protein 2 homolog B",
  "gene_symbol": "ATG2B",
  "term_id": "GO:0000422",
  "term_label": "autophagy of mitochondrion",
  "gene": "UniProtKB:Q96BY7"
}